{
  "term_id": "GO:0047220",
  "gene_symbol": "B3GALT6",
  "gene": "UniProtKB:Q96L58",
  "gene_name": "Beta-1,3-galactosyltransferase 6",
  "term_label": "galactosylxylosylprotein 3-beta-galactosyltransferase activity"
}